propionyl-CoA carboxylase activity [GO:0004658] (molecular function) Also known as: PCCase activity, propanoyl-CoA:carbon-dioxide ligase (ADP-forming), propionyl coenzyme A carboxylase activity Definition: Catalysis of the reaction: ATP + propanoyl-CoA + HCO3- = ADP + phosphate + (S)-methylmalonyl-CoA. Relationships: is a type of CoA carboxylase activity [GO:0016421] Sources: EC:6.4.1.3